{
  "term_label": "preribosome, large subunit precursor",
  "gene_symbol": "PPAN",
  "gene": "UniProtKB:Q9NQ55",
  "gene_name": "Suppressor of SWI4 1 homolog",
  "term_id": "GO:0030687"
}